interleukin-24 receptor binding [GO:0045520] (molecular function) Also known as: IL-24, interleukin-24 receptor ligand Sources: GOC:go_curators Definition: Binding to an interleukin-24 receptor. Relationships: is a type of GO:0005126